peptidyl-dipeptidase activity [GO:0008241] (molecular function) Relationships: is a type of GO:0008238 Sources: EC:3.4.15.-, GOC:mb Definition: Catalysis of the release of C-terminal dipeptides from a polypeptide chain. Regulation: negatively regulated by peptidyl-dipeptidase inhibitor activity [GO:0060422]